chorionic trophoblast cell development [GO:0060719] (biological process) Definition: The process whose specific outcome is the progression of the chorionic trophoblast over time, from its formation to the mature structure. Cell development does not include the steps involved in committing a cell to a specific fate. Relationships: is a type of cell development [GO:0048468]; is part of chorionic trophoblast cell differentiation [GO:0060718] Sources: CL:0011101, GOC:16983341, GOC:dph